{
  "gene_symbol": "DNAJC6",
  "gene_name": "Putative tyrosine-protein phosphatase auxilin",
  "gene": "UniProtKB:O75061",
  "term_label": "vesicle",
  "term_id": "GO:0031982"
}